{
  "gene": "UniProtKB:Q9NQC7",
  "term_label": "necroptotic process",
  "term_id": "GO:0070266",
  "gene_symbol": "CYLD",
  "gene_name": "Ubiquitin carboxyl-terminal hydrolase CYLD"
}